{
  "gene_name": "Lymphocyte cytosolic protein 2",
  "gene_symbol": "LCP2",
  "gene": "UniProtKB:Q13094",
  "term_id": "GO:0036398",
  "term_label": "TCR signalosome"
}